{
  "gene": "UniProtKB:A0A0B4J241",
  "term_label": "response to bacterium",
  "gene_name": "T cell receptor alpha variable 13-1",
  "term_id": "GO:0009617",
  "gene_symbol": "TRAV13-1"
}